bract development [GO:0010432] (biological process) References: PMID:16554366 Sources: GOC:tb, PO:0009055 Relationships: is a type of phyllome development [GO:0048827] Definition: The process whose specific outcome is the progression of the bract over time, from its formation to the mature structure. A bract is a leaf, usually different in form from the foliage leaves, subtending a flower or inflorescence.